{
  "term_label": "embryonic organ development",
  "gene_symbol": "PBX3",
  "gene": "UniProtKB:P40426",
  "term_id": "GO:0048568",
  "gene_name": "Pre-B-cell leukemia transcription factor 3"
}